{
  "term_id": "GO:0005184",
  "gene": "UniProtKB:O15130",
  "term_label": "neuropeptide hormone activity",
  "gene_symbol": "NPFF",
  "gene_name": "Pro-FMRFamide-related neuropeptide FF"
}